{
  "gene_name": "TBC1 domain family member 3C",
  "gene_symbol": "TBC1D3C",
  "term_id": "UNKNOWN:0002",
  "term_label": "Unknown biological process",
  "gene": "UniProtKB:Q6IPX1"
}